{
  "term_id": "GO:0016607",
  "gene_symbol": "PLCB1",
  "gene": "UniProtKB:Q9NQ66",
  "gene_name": "1-phosphatidylinositol 4,5-bisphosphate phosphodiesterase beta-1",
  "term_label": "nuclear speck"
}